negative regulation of cytokine production [GO:0001818] (biological process) Relationships: is a type of regulation of cytokine production [GO:0001817]; is a type of negative regulation of gene expression [GO:0010629]; is a type of negative regulation of multicellular organismal process [GO:0051241]; negatively regulates GO:0001816 Subtypes: negative regulation of cytokine production involved in immune response [GO:0002719], GO:0032480, negative regulation of chemokine production [GO:0032682], negative regulation of connective tissue growth factor production [GO:0032683], negative regulation of granulocyte macrophage colony-stimulating factor production [GO:0032685], negative regulation of hepatocyte growth factor production [GO:0032686], negative regulation of type II interferon production [GO:0032689], negative regulation of interleukin-1 production [GO:0032692], negative regulation of interleukin-10 production [GO:0032693], negative regulation of interleukin-11 production [GO:0032694], negative regulation of interleukin-12 production [GO:0032695], negative regulation of interleukin-13 production [GO:0032696], negative regulation of interleukin-15 production [GO:0032698], negative regulation of interleukin-16 production [GO:0032699], negative regulation of interleukin-17 production [GO:0032700], GO:0032701, negative regulation of interleukin-19 production [GO:0032702], negative regulation of interleukin-2 production [GO:0032703], GO:0032704, GO:0032705, GO:0032706, negative regulation of interleukin-23 production [GO:0032707], GO:0032708, negative regulation of interleukin-25 production [GO:0032709], GO:0032710, negative regulation of interleukin-27 production [GO:0032711], negative regulation of interleukin-3 production [GO:0032712], GO:0032713, negative regulation of interleukin-5 production [GO:0032714], negative regulation of interleukin-6 production [GO:0032715], GO:0032716, GO:0032717, negative regulation of interleukin-9 production [GO:0032718], GO:0034345, GO:0070755, negative regulation of transforming growth factor beta production [GO:0071635], negative regulation of fibroblast growth factor production [GO:0090272], negative regulation of interleukin-33 production [GO:0150128], negative regulation of interleukin-37 production [GO:0150138], negative regulation of interleukin-34 production [GO:0150159], negative regulation of interleukin-32 production [GO:0150190], negative regulation of cytokine production involved in inflammatory response [GO:1900016], negative regulation of glial cell-derived neurotrophic factor production [GO:1900167], negative regulation of macrophage colony-stimulating factor production [GO:1901257], negative regulation of tumor necrosis factor superfamily cytokine production [GO:1903556], GO:1904046, GO:1904471 Sources: GOC:add, ISBN:0781735149 Also known as: down regulation of cytokine biosynthetic process, down regulation of cytokine production, down-regulation of cytokine biosynthetic process, down-regulation of cytokine production, downregulation of cytokine biosynthetic process, downregulation of cytokine production, negative regulation of cytokine anabolism, negative regulation of cytokine biosynthesis, negative regulation of cytokine formation, negative regulation of cytokine synthesis, inhibition of cytokine biosynthetic process, inhibition of cytokine production, negative regulation of cytokine biosynthetic process, negative regulation of cytokine secretion Definition: Any process that stops, prevents, or reduces the rate of production of a cytokine.